{
  "gene_name": "Piwi-like protein 1",
  "gene": "UniProtKB:Q96J94",
  "term_id": "GO:0007283",
  "gene_symbol": "PIWIL1",
  "term_label": "spermatogenesis"
}